{
  "gene_symbol": "DENND4B",
  "gene": "UniProtKB:O75064",
  "term_id": "GO:0031410",
  "term_label": "cytoplasmic vesicle",
  "gene_name": "DENN domain-containing protein 4B"
}